kaempferol O-glucoside biosynthetic process [GO:0033330] (biological process) Also known as: kaempferol O-glucoside anabolism, kaempferol O-glucoside biosynthesis, kaempferol O-glucoside formation, kaempferol O-glucoside synthesit Definition: The chemical reactions and pathways leading to the formation of O-glucosylated derivatives of kaempferol. Sources: GOC:mah, MetaCyc:PWY-5320 Relationships: is a type of flavone biosynthetic process [GO:0051553]; is a type of beta-glucoside biosynthetic process [GO:1901806]